{
  "gene_name": "Beta-defensin 130B",
  "gene": "UniProtKB:P0DP73",
  "term_id": "GO:0042056",
  "term_label": "chemoattractant activity",
  "gene_symbol": "DEFB130B"
}